{
  "gene": "UniProtKB:Q96K37",
  "gene_symbol": "SLC35E1",
  "term_id": "GO:0055085",
  "term_label": "transmembrane transport",
  "gene_name": "Solute carrier family 35 member E1"
}